{
  "term_id": "GO:0000118",
  "gene_name": "Lysine-specific demethylase 3B",
  "term_label": "histone deacetylase complex",
  "gene_symbol": "KDM3B",
  "gene": "UniProtKB:Q7LBC6"
}